{
  "gene_symbol": "DAZ1",
  "gene": "UniProtKB:Q9NQZ3",
  "term_id": "GO:0070935",
  "term_label": "3'-UTR-mediated mRNA stabilization",
  "gene_name": "Deleted in azoospermia protein 1"
}